N-methyl nucleosidase activity [GO:0033960] (molecular function) Also known as: 7-methylxanthosine nucleosidase activity, 7-methylxanthosine ribohydrolase activity, N-MeNase activity, N-methyl nucleoside hydrolase activity, methylpurine nucleosidase activity Sources: EC:3.2.2.25, RHEA:10880 Definition: Catalysis of the reaction: 7-methylxanthosine + H2O = 7-methylxanthine + H+ + ribofuranose. Relationships: is_a hydrolase activity, hydrolyzing N-glycosyl compounds [GO:0016799]